{
  "term_id": "UNKNOWN:0003",
  "gene_symbol": "TP53TG5",
  "term_label": "Unknown cellular component",
  "gene_name": "TP53-target gene 5 protein",
  "gene": "UniProtKB:Q9Y2B4"
}